hydrogenase (acceptor) activity [GO:0033748] (molecular function) Relationships: is a type of oxidoreductase activity, acting on hydrogen as donor [GO:0016695] Definition: Catalysis of the reaction: H2 + A = AH2. Also known as: H2 producing hydrogenase activity, hydrogen-lyase activity, hydrogenlyase activity, uptake hydrogenase activity, hydrogen:(acceptor) oxidoreductase activity, hydrogen:acceptor oxidoreductase activity Sources: EC:1.12.99.6